{
  "gene": "UniProtKB:P09603",
  "term_id": "GO:0005125",
  "gene_name": "Macrophage colony-stimulating factor 1",
  "term_label": "cytokine activity",
  "gene_symbol": "CSF1"
}